{
  "gene": "UniProtKB:O75112",
  "term_label": "muscle structure development",
  "gene_symbol": "LDB3",
  "gene_name": "LIM domain-binding protein 3",
  "term_id": "GO:0061061"
}